{
  "gene_name": "Uncharacterized protein C11orf97",
  "gene": "UniProtKB:A0A1B0GVM6",
  "gene_symbol": "C11orf97",
  "term_id": "GO:0097546",
  "term_label": "ciliary base"
}